{
  "gene": "UniProtKB:Q16678",
  "term_id": "GO:0009404",
  "term_label": "toxin metabolic process",
  "gene_symbol": "CYP1B1",
  "gene_name": "Cytochrome P450 1B1"
}